{
  "term_id": "GO:0005737",
  "term_label": "cytoplasm",
  "gene_name": "Cilia- and flagella-associated protein 65",
  "gene_symbol": "CFAP65",
  "gene": "UniProtKB:Q6ZU64"
}